GLI-SUFU complex [GO:1990788] (cellular component) References: PMID:24311597 Sources: GOC:bhm Note: An example of this is SUFU in human (Q9UMX1) in PMID:24311597 (inferred from direct assay). Relationships: is a type of protein-containing complex [GO:0032991]; is part of cytosol [GO:0005829] Definition: A protein repressing GLI's transcription factor activity when SMO signaling is inactive. Upon ligand binding to the upstream receptor PTC (Patched) GLI dissociates from SUFU and activates transcription of hedgehog-target genes. In mammals it consists of SUFU and one of the GLI family proteins.